{
  "term_label": "voltage-gated potassium channel activity",
  "gene": "UniProtKB:Q9ULD8",
  "gene_symbol": "KCNH3",
  "gene_name": "Potassium voltage-gated channel subfamily H member 3",
  "term_id": "GO:0005249"
}